{
  "gene_symbol": "LINC02915",
  "gene": "UniProtKB:Q8N8G6",
  "term_id": "UNKNOWN:0001",
  "gene_name": "Putative uncharacterized protein encoded by LINC02915",
  "term_label": "Unknown molecular function"
}